{
  "gene": "UniProtKB:Q8NGZ0",
  "gene_name": "Olfactory receptor 2AJ1",
  "term_label": "plasma membrane",
  "gene_symbol": "OR2AJ1",
  "term_id": "GO:0005886"
}